{
  "gene_symbol": "TEX37",
  "gene": "UniProtKB:Q96LM6",
  "term_label": "Unknown molecular function",
  "gene_name": "Testis-expressed sequence 37 protein",
  "term_id": "UNKNOWN:0001"
}